{
  "term_id": "UNKNOWN:0002",
  "gene": "UniProtKB:O60303",
  "gene_symbol": "KATNIP",
  "term_label": "Unknown biological process",
  "gene_name": "Katanin-interacting protein"
}